{
  "gene": "UniProtKB:P20711",
  "term_label": "serotonin biosynthetic process",
  "term_id": "GO:0042427",
  "gene_name": "Aromatic-L-amino-acid decarboxylase",
  "gene_symbol": "DDC"
}